{
  "term_label": "Unknown cellular component",
  "term_id": "UNKNOWN:0003",
  "gene_symbol": "NAV2",
  "gene_name": "Neuron navigator 2",
  "gene": "UniProtKB:Q8IVL1"
}